positive regulation of defense response to bacterium [GO:1900426] (biological process) Relationships: is a type of positive regulation of response to biotic stimulus [GO:0002833]; is a type of positive regulation of defense response [GO:0031349]; is a type of GO:0032103; is a type of regulation of defense response to bacterium [GO:1900424]; positively regulates defense response to bacterium [GO:0042742] Subtypes: GO:0002803, positive regulation of peptidoglycan recognition protein signaling pathway [GO:0061059], positive regulation of neutrophil mediated killing of bacterium [GO:0070962] References: PMID:22346749 Sources: GOC:TermGenie Definition: Any process that activates or increases the frequency, rate or extent of defense response to bacterium. Also known as: activation of defence response to bacteria, activation of defence response to bacterium, activation of defense response to bacteria, positive regulation of defence response to bacteria, positive regulation of defence response to bacterium, positive regulation of defense response to bacteria, up regulation of defence response to bacteria, up regulation of defence response to bacterium, up regulation of defense response to bacteria, up regulation of defense response to bacterium, up-regulation of defence response to bacteria, up-regulation of defence response to bacterium, up-regulation of defense response to bacteria, up-regulation of defense response to bacterium, upregulation of defence response to bacteria, upregulation of defence response to bacterium, upregulation of defense response to bacteria, upregulation of defense response to bacterium, activation of defense response to bacterium, activation of resistance response to pathogenic bacteria, activation of resistance response to pathogenic bacterium, positive regulation of defense response to bacterium, incompatible interaction, activation of antibacterial peptide activity, positive regulation of antibacterial peptide activity, up regulation of antibacterial peptide activity, up-regulation of antibacterial peptide activity, upregulation of antibacterial peptide activity